{
  "term_id": "GO:0030027",
  "gene_symbol": "AMOT",
  "gene": "UniProtKB:Q4VCS5",
  "term_label": "lamellipodium",
  "gene_name": "Angiomotin"
}